prostaglandin transmembrane transporter activity [GO:0015132] (molecular function) Relationships: is a type of GO:0071714; is part of prostaglandin transport [GO:0015732] Definition: Enables the transfer of prostaglandins from one side of a membrane to the other. A prostaglandin is any of a group of biologically active metabolites which contain a cyclopentane ring due to the formation of a bond between two carbons of a fatty acid. They have a wide range of biological activities. Sources: GOC:ai Also known as: prostaglandin/thromboxane transporter activity